stomatal complex development [GO:0010374] (biological process) Regulation: regulated by regulation of stomatal complex development [GO:2000038]; negatively regulated by negative regulation of stomatal complex development [GO:2000122]; positively regulated by positive regulation of stomatal complex development [GO:2000123] Relationships: is a type of post-embryonic development [GO:0009791]; is a type of GO:0090558 References: PMID:17259259 Definition: The process whose specific outcome is the progression of the stomatal complex over time from its formation to the mature structure. The stomatal complex is the stomatal guard cells and their associated epidermal cells.